receptor-mediated virion attachment to host cell [GO:0046813] (biological process) Relationships: is a type of virion attachment to host cell [GO:0019062]; has part signaling receptor binding [GO:0005102] Sources: ISBN:0879694971 Regulation: regulated by regulation of receptor-mediated virion attachment to host cell [GO:1902734]; RO_0002212 by GO:1902735; positively regulated by positive regulation of receptor-mediated virion attachment to host cell [GO:1902736] Definition: The process by which a virion attaches to a host cell by binding to a receptor on the host cell surface. Also known as: virion attachment, binding of host cell surface receptor Subtypes: entry receptor-mediated virion attachment to host cell [GO:0098670], adhesion receptor-mediated virion attachment to host cell [GO:0098671]